{
  "gene": "UniProtKB:Q08629",
  "term_id": "GO:0031012",
  "gene_symbol": "SPOCK1",
  "gene_name": "Testican-1",
  "term_label": "extracellular matrix"
}